{
  "term_id": "GO:0045095",
  "term_label": "keratin filament",
  "gene": "UniProtKB:P08779",
  "gene_name": "Keratin, type I cytoskeletal 16",
  "gene_symbol": "KRT16"
}